{
  "term_id": "GO:0005737",
  "term_label": "cytoplasm",
  "gene_name": "Cadherin-1",
  "gene_symbol": "CDH1",
  "gene": "UniProtKB:P12830"
}